maltodextrin transmembrane transport [GO:0042956] (biological process) Also known as: maltodextrin transport Relationships: is a type of dextrin transport [GO:0042955] Sources: GOC:jl Definition: The directed movement of maltodextrin, any polysaccharide of glucose residues in beta-(1,4) linkage, across a membrane.